filopodium tip [GO:0032433] (cellular component) Definition: The end of a filopodium distal to the body of the cell. Sources: GOC:mah Relationships: is a type of cellular anatomical structure [GO:0110165]; is part of filopodium [GO:0030175]